host thylakoid [GO:0044159] (cellular component) Relationships: is a type of host intracellular organelle [GO:0033647] Definition: A membranous cellular structure within the host cell that bears the photosynthetic pigments in plants, algae, and cyanobacteria. In cyanobacteria thylakoids are of various shapes and are attached to, or continuous with, the host plasma membrane. In eukaryotic host cells they are flattened, membrane-bounded disk-like structures located in the chloroplasts; in the chloroplasts of higher plants the thylakoids form dense stacks called grana. Isolated thylakoid preparations can carry out photosynthetic electron transport and the associated phosphorylation. Sources: GOC:rph